plasma membrane raft localization [GO:0044856] (biological process) Sources: GOC:jl Subtypes: GO:0044855 Definition: Any process in which plasma membrane rafts are transported to, or maintained in, a specific location. Relationships: is a type of plasma membrane organization [GO:0007009]; is a type of membrane raft localization [GO:0051665]